{
  "gene_name": "Ankyrin repeat domain-containing protein SOWAHA",
  "term_id": "UNKNOWN:0003",
  "term_label": "Unknown cellular component",
  "gene_symbol": "SOWAHA",
  "gene": "UniProtKB:Q2M3V2"
}